{
  "term_id": "GO:0005085",
  "gene": "UniProtKB:Q9Y4F1",
  "gene_name": "FERM, ARHGEF and pleckstrin domain-containing protein 1",
  "gene_symbol": "FARP1",
  "term_label": "guanyl-nucleotide exchange factor activity"
}